{
  "gene_symbol": "SNCA",
  "gene": "UniProtKB:P37840",
  "term_label": "axon terminus",
  "gene_name": "Alpha-synuclein",
  "term_id": "GO:0043679"
}